{
  "term_id": "GO:0005737",
  "gene_name": "Oncomodulin-1",
  "term_label": "cytoplasm",
  "gene_symbol": "OCM",
  "gene": "UniProtKB:P0CE72"
}